{
  "gene_name": "Histidine--tRNA ligase, mitochondrial",
  "gene_symbol": "HARS2",
  "term_id": "GO:0004821",
  "gene": "UniProtKB:P49590",
  "term_label": "histidine-tRNA ligase activity"
}